{
  "term_label": "Unknown cellular component",
  "gene_symbol": "HSPA12B",
  "term_id": "UNKNOWN:0003",
  "gene_name": "Heat shock 70 kDa protein 12B",
  "gene": "UniProtKB:Q96MM6"
}